{
  "gene_symbol": "CSNK1A1",
  "gene": "UniProtKB:P48729",
  "term_label": "negative regulation of canonical Wnt signaling pathway",
  "gene_name": "Casein kinase I isoform alpha",
  "term_id": "GO:0090090"
}